transcription elongation by mitochondrial RNA polymerase [GO:0006392] (biological process) Also known as: RNA elongation from mitochondrial promoter, transcription elongation from mitochondrial promoter Definition: The extension of an RNA molecule after transcription initiation and promoter clearance at mitochondrial promoter by the addition of ribonucleotides catalyzed by a mitchondrial RNA polymerase. Sources: GOC:mah, GOC:txnOH Relationships: is a type of mitochondrial RNA metabolic process [GO:0000959]; is a type of DNA-templated transcription elongation [GO:0006354]; BFO_0000050 mitochondrial transcription [GO:0006390]